fatty acid beta-oxidation using acyl-CoA dehydrogenase [GO:0033539] (biological process) Definition: A fatty acid beta-oxidation pathway in which the initial step of each oxidation cycle, which converts an acyl-CoA to a trans-2-enoyl-CoA, is catalyzed by acyl-CoA dehydrogenase; the electrons removed by oxidation pass through the respiratory chain to oxygen and leave H2O as the product. Fatty acid beta-oxidation begins with the addition of coenzyme A to a fatty acid, and ends when only two or three carbons remain (as acetyl-CoA or propionyl-CoA respectively). Regulation: regulated by regulation of fatty acid beta-oxidation using acyl-CoA dehydrogenase [GO:1904735]; RO_0002212 by GO:1904736; positively regulated by GO:1904737 Sources: GOC:mah, MetaCyc:FAO-PWY Relationships: is a type of fatty acid beta-oxidation [GO:0006635]; has part GO:0003995